{
  "gene_name": "Peptide YY",
  "gene": "UniProtKB:P10082",
  "gene_symbol": "PYY",
  "term_id": "GO:0007631",
  "term_label": "feeding behavior"
}